{
  "term_label": "mitochondrial promoter sequence-specific DNA binding",
  "gene": "UniProtKB:O00411",
  "gene_symbol": "POLRMT",
  "term_id": "GO:0001018",
  "gene_name": "DNA-directed RNA polymerase, mitochondrial"
}